{
  "gene": "UniProtKB:Q6S545",
  "gene_name": "POTE ankyrin domain family member H",
  "gene_symbol": "POTEH",
  "term_label": "Unknown cellular component",
  "term_id": "UNKNOWN:0003"
}